negative regulation of thyroid hormone receptor signaling pathway [GO:0002156] (biological process) Relationships: is a type of GO:0002155; is a type of GO:1902532; RO_0002212 thyroid hormone receptor signaling pathway [GO:0002154] Also known as: negative regulation of thyroid hormone mediated signaling pathway, negative regulation of thyroid hormone mediated signalling pathway Sources: GOC:hjd Definition: Any process that stops, prevents, or reduces the frequency, rate or extent of thyroid hormone mediated signaling pathway.